{
  "gene_name": "Interferon lambda-3",
  "term_id": "GO:0005102",
  "gene": "UniProtKB:Q8IZI9",
  "term_label": "signaling receptor binding",
  "gene_symbol": "IFNL3"
}